{
  "term_id": "UNKNOWN:0002",
  "gene_name": "Retinoblastoma-binding protein 5",
  "gene": "UniProtKB:Q15291",
  "gene_symbol": "RBBP5",
  "term_label": "Unknown biological process"
}